establishment of dense core granule localization [GO:0032256] (biological process) Definition: The directed movement of a dense core granule to a specific location. Also known as: establishment of dense core granule localisation, establishment of dense core vesicle localization Sources: GOC:mah Relationships: is a type of GO:0032254; is part of dense core granule localization [GO:0032253]